mitochondrial matrix [GO:0005759] (cellular component) Sources: GOC:as, ISBN:0198506732 Also known as: mitochondrial lumen, mitochondrial stroma Definition: The gel-like material, with considerable fine structure, that lies in the matrix space, or lumen, of a mitochondrion. It contains the enzymes of the tricarboxylic acid cycle and, in some organisms, the enzymes concerned with fatty acid oxidation. Relationships: is a type of intracellular organelle lumen [GO:0070013]; is part of mitochondrion [GO:0005739]